{
  "gene_name": "Neutrophil defensin 3",
  "gene_symbol": "DEFA3",
  "term_id": "GO:0045087",
  "term_label": "innate immune response",
  "gene": "UniProtKB:P59666"
}